{
  "gene_symbol": "CYP2A6",
  "term_label": "heme binding",
  "term_id": "GO:0020037",
  "gene": "UniProtKB:P11509",
  "gene_name": "Cytochrome P450 2A6"
}